{
  "term_id": "GO:0007155",
  "gene_name": "Sialic acid-binding Ig-like lectin 7",
  "gene_symbol": "SIGLEC7",
  "term_label": "cell adhesion",
  "gene": "UniProtKB:Q9Y286"
}